{
  "term_label": "retrograde vesicle-mediated transport, Golgi to endoplasmic reticulum",
  "gene_name": "Sec1 family domain-containing protein 1",
  "gene": "UniProtKB:Q8WVM8",
  "gene_symbol": "SCFD1",
  "term_id": "GO:0006890"
}